positive regulation of mesodermal cell differentiation [GO:1905772] (biological process) Also known as: positive regulation of mesoderm cell differentiation, up regulation of mesoderm cell differentiation, up regulation of mesodermal cell differentiation, up-regulation of mesoderm cell differentiation, up-regulation of mesodermal cell differentiation, upregulation of mesoderm cell differentiation, upregulation of mesodermal cell differentiation, activation of mesoderm cell differentiation, activation of mesodermal cell differentiation Definition: Any process that activates or increases the frequency, rate or extent of mesodermal cell differentiation. Relationships: is a type of positive regulation of cell differentiation [GO:0045597]; is a type of regulation of mesodermal cell differentiation [GO:1905770]; positively regulates mesodermal cell differentiation [GO:0048333] Subtypes: positive regulation of mesodermal cell fate specification [GO:0048337] References: PMID:23765923 Sources: GOC:BHF, GOC:BHF_miRNA, GOC:TermGenie, GOC:rph, GO_REF:0000058